{
  "gene_name": "Rho-associated protein kinase 1",
  "gene": "UniProtKB:Q13464",
  "term_label": "embryonic morphogenesis",
  "gene_symbol": "ROCK1",
  "term_id": "GO:0048598"
}